{
  "gene": "UniProtKB:Q96F44",
  "term_id": "GO:0046597",
  "gene_name": "E3 ubiquitin-protein ligase TRIM11",
  "term_label": "host-mediated suppression of symbiont invasion",
  "gene_symbol": "TRIM11"
}